{
  "gene": "UniProtKB:Q14318",
  "term_id": "GO:0012505",
  "gene_symbol": "FKBP8",
  "gene_name": "Peptidyl-prolyl cis-trans isomerase FKBP8",
  "term_label": "endomembrane system"
}